{
  "term_label": "kinesin complex",
  "gene": "UniProtKB:O43896",
  "gene_name": "Kinesin-like protein KIF1C",
  "term_id": "GO:0005871",
  "gene_symbol": "KIF1C"
}